{
  "term_id": "GO:0005634",
  "gene_symbol": "MSH2",
  "gene_name": "DNA mismatch repair protein Msh2",
  "gene": "UniProtKB:P43246",
  "term_label": "nucleus"
}